sensory dendrite [GO:0071683] (CC) Relationships: is a type of GO:0030425 Sources: GOC:dos, GOC:kmv, GOC:mah Definition: A dendrite that is found on a sensory neuron, and directly transduces a sensory signal from the sensory neuron to another neuron.